{
  "gene": "UniProtKB:P18031",
  "term_id": "GO:0070373",
  "gene_symbol": "PTPN1",
  "gene_name": "Tyrosine-protein phosphatase non-receptor type 1",
  "term_label": "negative regulation of ERK1 and ERK2 cascade"
}